{
  "gene_name": "Arylsulfatase A",
  "term_label": "arylsulfatase activity",
  "term_id": "GO:0004065",
  "gene": "UniProtKB:P15289",
  "gene_symbol": "ARSA"
}